{
  "term_label": "establishment or maintenance of epithelial cell apical/basal polarity",
  "gene_symbol": "DLG1",
  "term_id": "GO:0045197",
  "gene": "UniProtKB:Q12959",
  "gene_name": "Disks large homolog 1"
}